{
  "gene": "UniProtKB:O43609",
  "term_label": "protein kinase inhibitor activity",
  "gene_symbol": "SPRY1",
  "term_id": "GO:0004860",
  "gene_name": "Protein sprouty homolog 1"
}